{
  "gene": "UniProtKB:Q99436",
  "term_id": "GO:0005634",
  "gene_name": "Proteasome subunit beta type-7",
  "term_label": "nucleus",
  "gene_symbol": "PSMB7"
}